{
  "term_id": "GO:0042742",
  "gene": "UniProtKB:O15263",
  "gene_name": "Defensin beta 4A",
  "gene_symbol": "DEFB4B",
  "term_label": "defense response to bacterium"
}